Fc-gamma receptor III complex [GO:0033001] (cellular component) References: PMID:11244038, PMID:12413532 Sources: GOC:add, ISBN:0781735149 Also known as: IgG receptor complex, immunoglobulin G receptor complex, FcgRIII complex Definition: A protein complex composed of an Fc-gamma RIII alpha chain and an Fc-epsilon RI gamma chain dimer with or without an Fc-epsilon RI beta chain and additional signaling components. The complex functions primarily as an activating receptor for IgG. Relationships: is a type of Fc receptor complex [GO:0032997]